{
  "gene_symbol": "C8B",
  "gene_name": "Complement component C8 beta chain",
  "term_id": "GO:0005615",
  "gene": "UniProtKB:P07358",
  "term_label": "extracellular space"
}